ATP:ADP adenylyltransferase activity [GO:0003877] (molecular function) Also known as: ATP adenylyltransferase activity, AP-4-A phosphorylase activity, adenine triphosphate adenylyltransferase activity, bis(5'-nucleosyl)-tetraphosphate phosphorylase (NDP-forming) activity, diadenosine 5',5'''-P(1),P(4)-tetraphosphate phosphorylase activity, diadenosine 5',5'''-P1,P4-tetraphosphate alphabeta-phosphorylase (ADP-forming), diadenosine 5',5'''-P1,P4-tetraphosphate phosphorylase activity, diadenosinetetraphosphate alpha-beta-phosphorylase activity, diadenosinetetraphosphate alphabeta-phosphorylase activity, dinucleoside oligophosphate alphabeta-phosphorylase activity Relationships: is a type of adenylyltransferase activity [GO:0070566] Sources: EC:2.7.7.53 Definition: Catalysis of the reaction: ADP + ATP = phosphate + P(1),P(4)-bis(5'-adenosyl)tetraphosphate.